chalcone catabolic process [GO:0046280] (biological process) Definition: The chemical reactions and pathways resulting in the breakdown of chalcone, phenyl steryl ketone or its hydroxylated derivatives. Sources: GOC:ai Also known as: chalcone breakdown, chalcone catabolism, chalcone degradation Relationships: is a type of ketone catabolic process [GO:0042182]; is a type of phenylpropanoid catabolic process [GO:0046271]; is a type of olefinic compound catabolic process [GO:0120256]